{
  "gene": "UniProtKB:A6NCN2",
  "gene_symbol": "KRT87P",
  "term_label": "Unknown biological process",
  "term_id": "UNKNOWN:0002",
  "gene_name": "Putative keratin-87 protein"
}